{
  "term_id": "GO:0070665",
  "gene_symbol": "CSF2RB",
  "gene": "UniProtKB:P32927",
  "gene_name": "Cytokine receptor common subunit beta",
  "term_label": "positive regulation of leukocyte proliferation"
}